{
  "gene_name": "Calcium homeostasis modulator protein 4",
  "gene_symbol": "CALHM4",
  "gene": "UniProtKB:Q5JW98",
  "term_id": "UNKNOWN:0002",
  "term_label": "Unknown biological process"
}